{
  "term_label": "cyclin-dependent protein kinase holoenzyme complex",
  "gene": "UniProtKB:Q16589",
  "gene_symbol": "CCNG2",
  "gene_name": "Cyclin-G2",
  "term_id": "GO:0000307"
}